positive regulation of mononuclear cell migration [GO:0071677] (biological process) Also known as: up regulation of mononuclear cell migration, up-regulation of mononuclear cell migration, upregulation of mononuclear cell migration, activation of mononuclear cell migration, stimulation of mononuclear cell migration Sources: GOC:mah Relationships: is a type of positive regulation of leukocyte migration [GO:0002687]; is a type of regulation of mononuclear cell migration [GO:0071675]; positively regulates GO:0071674 Subtypes: GO:0090026, positive regulation of macrophage migration [GO:1905523], GO:2000403, GO:2000439, positive regulation of dendritic cell chemotaxis [GO:2000510] Definition: Any process that increases the rate, frequency or extent of mononuclear cell migration. Mononuclear cell migration is the movement of a mononuclear cell within or between different tissues and organs of the body.